{
  "gene": "UniProtKB:P28223",
  "gene_symbol": "HTR2A",
  "term_id": "GO:0009410",
  "gene_name": "5-hydroxytryptamine receptor 2A",
  "term_label": "response to xenobiotic stimulus"
}